{
  "term_id": "GO:0017099",
  "gene": "UniProtKB:P49748",
  "gene_symbol": "ACADVL",
  "gene_name": "Very long-chain specific acyl-CoA dehydrogenase, mitochondrial",
  "term_label": "very-long-chain fatty acyl-CoA dehydrogenase activity"
}